{
  "gene": "UniProtKB:O14977",
  "gene_name": "Antizyme inhibitor 1",
  "gene_symbol": "AZIN1",
  "term_id": "GO:0042978",
  "term_label": "ornithine decarboxylase activator activity"
}